{
  "gene_name": "Microsomal triglyceride transfer protein large subunit",
  "gene": "UniProtKB:P55157",
  "term_id": "GO:0005548",
  "term_label": "phospholipid transporter activity",
  "gene_symbol": "MTTP"
}